{
  "term_label": "nucleus",
  "term_id": "GO:0005634",
  "gene_symbol": "ZNF286A",
  "gene_name": "Zinc finger protein 286A",
  "gene": "UniProtKB:Q9HBT8"
}